vascular endothelial growth factor receptor 2 binding [GO:0043184] (molecular function) Sources: GOC:st Relationships: is a type of vascular endothelial growth factor receptor binding [GO:0005172] Definition: Binding to a vascular endothelial growth factor receptor 2. Also known as: KDR binding, Flk-1 binding, VEGF receptor 2 binding, VEGFR 2 binding, kinase domain region binding